{
  "gene": "UniProtKB:Q6ZN57",
  "gene_name": "Zinc finger protein ZFP2",
  "term_id": "UNKNOWN:0003",
  "gene_symbol": "ZFP2",
  "term_label": "Unknown cellular component"
}